{
  "gene_name": "Heparin cofactor 2",
  "term_label": "serine-type endopeptidase inhibitor activity",
  "gene": "UniProtKB:P05546",
  "term_id": "GO:0004867",
  "gene_symbol": "SERPIND1"
}